{
  "term_label": "neuron projection development",
  "gene": "UniProtKB:Q6ZVF9",
  "gene_name": "G protein-regulated inducer of neurite outgrowth 3",
  "gene_symbol": "GPRIN3",
  "term_id": "GO:0031175"
}